{
  "gene_name": "Stathmin-2",
  "gene_symbol": "STMN2",
  "gene": "UniProtKB:Q93045",
  "term_label": "microtubule depolymerization",
  "term_id": "GO:0007019"
}